{
  "gene_symbol": "PPP1R9B",
  "gene": "UniProtKB:Q96SB3",
  "term_label": "neuron projection development",
  "gene_name": "Neurabin-2",
  "term_id": "GO:0031175"
}